regulation of central tolerance induction [GO:0002646] (biological process) Definition: Any process that modulates the frequency, rate, or extent of central tolerance induction. Sources: GOC:add Relationships: is a type of GO:0002643; regulates central tolerance induction [GO:0002508] Subtypes: GO:0002647, positive regulation of central tolerance induction [GO:0002648], regulation of central B cell tolerance induction [GO:0002895]